{
  "gene_name": "2'-deoxynucleoside 5'-phosphate N-hydrolase 1",
  "gene": "UniProtKB:O43598",
  "gene_symbol": "DNPH1",
  "term_label": "deoxyribonucleoside monophosphate catabolic process",
  "term_id": "GO:0009159"
}